{
  "term_id": "UNKNOWN:0001",
  "gene_symbol": "SHKBP1",
  "gene_name": "SH3KBP1-binding protein 1",
  "gene": "UniProtKB:Q8TBC3",
  "term_label": "Unknown molecular function"
}